O6-methyl-dGTP hydrolase activity [GO:0106433] (molecular function) References: PMID:30304478 Sources: RHEA:67600 Definition: Catalysis of the reaction O6-methyl-dGTP + H2O = O6-methyl-dGMP + diphosphate + H+. Relationships: is a type of hydrolase activity, acting on acid anhydrides, in phosphorus-containing anhydrides [GO:0016818]